{
  "term_id": "GO:0006508",
  "gene_name": "Chymotrypsin-like elastase family member 2B",
  "gene": "UniProtKB:P08218",
  "gene_symbol": "CELA2B",
  "term_label": "proteolysis"
}